{
  "gene": "UniProtKB:Q01831",
  "term_id": "GO:0003684",
  "gene_symbol": "XPC",
  "gene_name": "DNA repair protein complementing XP-C cells",
  "term_label": "damaged DNA binding"
}